{
  "term_id": "UNKNOWN:0003",
  "gene": "UniProtKB:P62166",
  "term_label": "Unknown cellular component",
  "gene_name": "Neuronal calcium sensor 1",
  "gene_symbol": "NCS1"
}